{
  "gene": "UniProtKB:Q8IWU6",
  "term_label": "extracellular space",
  "term_id": "GO:0005615",
  "gene_name": "Extracellular sulfatase Sulf-1",
  "gene_symbol": "SULF1"
}